{
  "gene": "UniProtKB:P13995",
  "term_label": "methenyltetrahydrofolate cyclohydrolase activity",
  "term_id": "GO:0004477",
  "gene_symbol": "MTHFD2",
  "gene_name": "Bifunctional methylenetetrahydrofolate dehydrogenase_cyclohydrolase, mitochondrial"
}